{
  "term_id": "GO:0008138",
  "gene": "UniProtKB:Q9UNI6",
  "gene_symbol": "DUSP12",
  "gene_name": "Dual specificity protein phosphatase 12",
  "term_label": "protein tyrosine/serine/threonine phosphatase activity"
}